{
  "gene_name": "Transmembrane protein 248",
  "gene": "UniProtKB:Q9NWD8",
  "term_label": "Unknown molecular function",
  "gene_symbol": "TMEM248",
  "term_id": "UNKNOWN:0001"
}